{
  "gene_symbol": "ZNRF3",
  "term_id": "GO:0090090",
  "gene": "UniProtKB:Q9ULT6",
  "term_label": "negative regulation of canonical Wnt signaling pathway",
  "gene_name": "E3 ubiquitin-protein ligase ZNRF3"
}